alphav-beta3 integrin-osteopontin complex [GO:0070029] (cellular component) Relationships: is a type of plasma membrane protein complex [GO:0098797] Definition: A protein complex that consists of an alphav-beta3 integrin complex bound to osteopontin. Also known as: ITGAV-ITGB3-SPP1 complex References: PMID:7532190